hydroxyisourate hydrolase activity [GO:0033971] (molecular function) Relationships: is a type of hydrolase activity, acting on carbon-nitrogen (but not peptide) bonds, in cyclic amides [GO:0016812] Definition: Catalysis of the reaction: 5-hydroxyisourate + H2O = 5-hydroxy-2-oxo-4-ureido-2,5-dihydro-1H-imidazole-5-carboxylate + H+. Sources: EC:3.5.2.17, RHEA:23736 Also known as: 5-hydroxyisourate amidohydrolase activity, 5-hydroxyisourate hydrolase activity, HIUHase activity